{
  "gene": "UniProtKB:Q12840",
  "gene_symbol": "KIF5A",
  "gene_name": "Kinesin heavy chain isoform 5A",
  "term_label": "anterograde dendritic transport of neurotransmitter receptor complex",
  "term_id": "GO:0098971"
}